{
  "term_label": "cytoplasm",
  "gene_symbol": "AKR7A2",
  "gene_name": "Aflatoxin B1 aldehyde reductase member 2",
  "term_id": "GO:0005737",
  "gene": "UniProtKB:O43488"
}